{
  "gene_name": "Sperm acrosome membrane-associated protein 4",
  "gene": "UniProtKB:Q8TDM5",
  "term_id": "UNKNOWN:0001",
  "gene_symbol": "SPACA4",
  "term_label": "Unknown molecular function"
}